{
  "term_label": "nucleolus",
  "gene_symbol": "RIOX1",
  "gene": "UniProtKB:Q9H6W3",
  "gene_name": "Ribosomal oxygenase 1",
  "term_id": "GO:0005730"
}